{
  "term_id": "UNKNOWN:0001",
  "term_label": "Unknown molecular function",
  "gene_name": "Centrosomal protein of 164 kDa",
  "gene": "UniProtKB:Q9UPV0",
  "gene_symbol": "CEP164"
}